symbiont-mediated suppression of host transcription [GO:0039653] (biological process) Definition: A process in which a symbiont inhibits or disrupts transcription of genes into mRNA in its host. For example, symbiont proteins can interfere with host RNA polymerase or with transcription factors. The host is defined as the larger of the organisms involved in a symbiotic interaction. Also known as: host transcription shut-off, host transcription shutoff by virus, suppression by virus of host DNA-dependent transcription, suppression by virus of host transcription Relationships: is a type of symbiont-mediated perturbation of host transcription [GO:0052026] Sources: VZ:1577 Subtypes: symbiont-mediated suppression of host mRNA transcription via inhibition of RNA polymerase II activity [GO:0039523]